establishment of meiotic sister chromatid cohesion [GO:0034089] (biological process) Definition: The process in which the sister chromatids of a replicated chromosome become joined along the entire length of the chromosome during S phase during a meiotic cell cycle. Sources: GOC:mah Relationships: is_a GO:0034085; is part of meiotic sister chromatid cohesion [GO:0051177]